{
  "gene_symbol": "HSPB1",
  "term_label": "protein refolding",
  "term_id": "GO:0042026",
  "gene": "UniProtKB:P04792",
  "gene_name": "Heat shock protein beta-1"
}